{
  "term_label": "potassium ion transmembrane transport",
  "gene_symbol": "KCNQ4",
  "gene": "UniProtKB:P56696",
  "gene_name": "Potassium voltage-gated channel subfamily KQT member 4",
  "term_id": "GO:0071805"
}